{
  "gene_symbol": "NF2",
  "gene_name": "Merlin",
  "term_id": "GO:1902966",
  "term_label": "positive regulation of protein localization to early endosome",
  "gene": "UniProtKB:P35240"
}